trans-synaptic signaling by endocannabinoid [GO:0099542] (biological process) Subtypes: retrograde trans-synaptic signaling by endocannabinoid [GO:0098921], trans-synaptic signaling by endocannabinoid, modulating synaptic transmission [GO:0099553] Definition: Cell-cell signaling in either direction across the synaptic cleft, mediated by an endocannabinoid ligand. Sources: GOC:dos Relationships: is a type of trans-synaptic signaling by lipid [GO:0099541]